{
  "term_id": "GO:0000462",
  "gene_name": "Nucleolar protein 10",
  "gene": "UniProtKB:Q9BSC4",
  "term_label": "maturation of SSU-rRNA from tricistronic rRNA transcript (SSU-rRNA, 5.8S rRNA, LSU-rRNA)",
  "gene_symbol": "NOL10"
}